{
  "term_label": "peroxisomal membrane",
  "gene_name": "E3 ubiquitin-protein ligase TRIM37",
  "gene": "UniProtKB:O94972",
  "gene_symbol": "TRIM37",
  "term_id": "GO:0005778"
}